{
  "term_label": "damaged DNA binding",
  "term_id": "GO:0003684",
  "gene_symbol": "ERCC2",
  "gene_name": "General transcription and DNA repair factor IIH helicase subunit XPD",
  "gene": "UniProtKB:P18074"
}